3-beta-hydroxy-Delta5-steroid dehydrogenase (NAD+) activity [GO:0003854] (molecular function) Sources: EC:1.1.1.145 Subtypes: cholesterol dehydrogenase (NAD+) activity [GO:0102294] Relationships: is a type of steroid dehydrogenase activity, acting on the CH-OH group of donors, NAD or NADP as acceptor [GO:0033764] Definition: Catalysis of the reaction: a 3-beta-hydroxy-Delta(5)-steroid + NAD+ = a 3-oxo-Delta(5)-steroid + NADH + H+. Also acts on on 3-beta-hydroxypregn-5-en-20-one to form progesterone. Also known as: 3beta-hydroxy-delta5-C27-steroid oxidoreductase, progesterone reductase activity, 3-beta-hydroxy-D5-steroid dehydrogenase activity, 3-beta-hydroxy-5-ene steroid dehydrogenase activity, 3beta-HSDH, 3beta-hydroxy steroid dehydrogenase/isomerase activity, 3beta-hydroxy-5-ene steroid dehydrogenase activity, 3beta-hydroxy-5-ene-steroid dehydrogenase activity, 3beta-hydroxy-5-ene-steroid oxidoreductase activity, 3beta-hydroxy-delta5-C27-steroid dehydrogenase/isomerase activity, 3beta-hydroxy-delta5-steroid dehydrogenase activity, 3beta-hydroxy-delta5-steroid:NAD+ 3-oxidoreductase activity, 5-ene-3-beta-hydroxysteroid dehydrogenase activity, delta5-3beta-hydroxysteroid dehydrogenase activity, steroid-delta5-3beta-ol dehydrogenase activity